{
  "term_id": "GO:0000421",
  "gene_name": "Protein associated with UVRAG as autophagy enhancer",
  "term_label": "autophagosome membrane",
  "gene": "UniProtKB:Q9H714",
  "gene_symbol": "RUBCNL"
}